{
  "term_label": "Unknown molecular function",
  "gene_symbol": "FAM72A",
  "gene_name": "Protein FAM72A",
  "term_id": "UNKNOWN:0001",
  "gene": "UniProtKB:Q5TYM5"
}